{
  "term_label": "potassium:proton antiporter activity",
  "gene": "UniProtKB:P19634",
  "term_id": "GO:0015386",
  "gene_name": "Sodium_hydrogen exchanger 1",
  "gene_symbol": "SLC9A1"
}